{
  "term_id": "GO:0006357",
  "term_label": "regulation of transcription by RNA polymerase II",
  "gene_symbol": "NKX2-4",
  "gene_name": "Homeobox protein Nkx-2.4",
  "gene": "UniProtKB:Q9H2Z4"
}